{
  "term_id": "GO:0098839",
  "gene_symbol": "CLSTN3",
  "gene": "UniProtKB:Q9BQT9",
  "gene_name": "Calsyntenin-3",
  "term_label": "postsynaptic density membrane"
}